{
  "gene_symbol": "AASDH",
  "gene_name": "Beta-alanine-activating enzyme",
  "term_label": "Unknown cellular component",
  "term_id": "UNKNOWN:0003",
  "gene": "UniProtKB:Q4L235"
}